{
  "term_id": "GO:0004930",
  "gene": "UniProtKB:P47775",
  "gene_symbol": "GPR12",
  "term_label": "G protein-coupled receptor activity",
  "gene_name": "G-protein coupled receptor 12"
}